{
  "term_label": "phosphatidylinositol 3-kinase complex",
  "term_id": "GO:0005942",
  "gene": "UniProtKB:O00329",
  "gene_symbol": "PIK3CD",
  "gene_name": "Phosphatidylinositol 4,5-bisphosphate 3-kinase catalytic subunit delta isoform"
}